protein insertion into ER membrane [GO:0045048] (biological process) Also known as: integral ER membrane protein localization, integral ER membrane protein positioning, localization of protein in ER membrane, positioning of protein in ER membrane, protein insertion into endoplasmic reticulum membrane, protein-ER insertion, protein-endoplasmic reticulum insertion Relationships: is a type of GO:0051205; is part of GO:0007029; BFO_0000050 protein localization to organelle [GO:0033365] Definition: The process that results in incorporation of a protein into an endoplasmic reticulum (ER) membrane. It depends on specific topogenic sequences of amino acids that ensure that a protein acquires the proper orientation during its insertion into the ER membrane. Sources: ISBN:0716731363 Subtypes: protein insertion into ER membrane by N-terminal cleaved signal sequence [GO:0045049], protein insertion into ER membrane by stop-transfer membrane-anchor sequence [GO:0045050], protein insertion into ER membrane by internal uncleaved signal-anchor sequence [GO:0045051], GO:0071816, multi-pass transmembrane protein insertion into ER membrane [GO:0160063]